regulation of RNA helicase activity [GO:1902280] (biological process) References: PMID:23721653 Sources: GOC:TermGenie, GOC:rb Relationships: is_a regulation of ATP-dependent activity [GO:0043462]; is a type of regulation of catalytic activity [GO:0050790]; regulates RNA helicase activity [GO:0003724] Also known as: regulation of ATP-dependent RNA helicase activity Definition: Any process that modulates the frequency, rate or extent of ATP-dependent RNA helicase activity.